TRIF-dependent toll-like receptor 4 signaling pathway [GO:0035667] (biological process) References: PMID:18641322, PMID:20511708 Sources: GOC:BHF Relationships: is a type of toll-like receptor 4 signaling pathway [GO:0034142]; is_a TRIF-dependent toll-like receptor signaling pathway [GO:0035666] Definition: The series of molecular signals initiated by a ligand binding to a toll-like 4 receptor where the TRIF adaptor mediates transduction of the signal. Toll-like 4 receptors are pattern recognition receptors that bind bacterial lipopolysaccharide (LPS) to initiate an innate immune response. Also known as: TRIF-dependent TLR4 signaling pathway, TRIF-dependent toll-like receptor 4 signalling pathway, Toll/IL-1 receptor (TIR) domain-containing adaptor-dependent TLR4 signaling pathway